{
  "term_label": "mitochondrion",
  "term_id": "GO:0005739",
  "gene": "UniProtKB:Q9Y3E2",
  "gene_name": "BolA-like protein 1",
  "gene_symbol": "BOLA1"
}